{
  "gene_name": "Protocadherin beta-4",
  "term_id": "GO:0005886",
  "gene": "UniProtKB:Q9Y5E5",
  "term_label": "plasma membrane",
  "gene_symbol": "PCDHB4"
}